flavonol 3-sulfotransferase activity [GO:0047894] (molecular function) Also known as: 3'-phosphoadenylyl-sulfate:quercetin 3-sulfotransferase activity, flavonol 3-sulphotransferase activity Sources: EC:2.8.2.25, RHEA:13453 Definition: Catalysis of the reaction: 3'-phospho-5'-adenylyl sulfate + quercetin = adenosine 3',5'-diphosphate + H+ + quercetin 3-sulfate. Relationships: is a type of sulfotransferase activity [GO:0008146]